female analia morphogenesis [GO:0048810] (biological process) References: PMID:11494318 Sources: GOC:mtg_sensu Definition: The process in which the anatomical structures of the analia of the female are generated and organized. The analia is the posterior-most vertral appendage that develops from the genital disc. An example of this process is found in Drosophila melanogaster. Relationships: is a type of analia morphogenesis [GO:0048809]; is part of GO:0045497